{
  "gene_name": "Centrosomal protein of 97 kDa",
  "gene": "UniProtKB:Q8IW35",
  "term_id": "GO:1902018",
  "gene_symbol": "CEP97",
  "term_label": "negative regulation of cilium assembly"
}